negative regulation of stress response to copper ion [GO:1903854] (BP) Definition: Any process that stops, prevents or reduces the frequency, rate or extent of stress response to copper ion. References: PMID:23437011 Sources: GOC:TermGenie, GOC:kmv, GO_REF:0000058 Relationships: is a type of negative regulation of response to stimulus [GO:0048585]; is a type of regulation of stress response to copper ion [GO:1903853]; negatively regulates stress response to copper ion [GO:1990169] Also known as: down regulation of response to copper ion stress, down regulation of stress response to copper ion, down-regulation of response to copper ion stress, down-regulation of stress response to copper ion, downregulation of response to copper ion stress, downregulation of stress response to copper ion, negative regulation of response to copper ion stress, inhibition of response to copper ion stress, inhibition of stress response to copper ion, down regulation of response to copper toxicity, down-regulation of response to copper toxicity, downregulation of response to copper toxicity, inhibition of response to copper toxicity, negative regulation of response to copper toxicity